{
  "gene_name": "Killer cell lectin-like receptor subfamily G member 2",
  "term_id": "UNKNOWN:0003",
  "gene_symbol": "KLRG2",
  "gene": "UniProtKB:A4D1S0",
  "term_label": "Unknown cellular component"
}